{
  "gene_symbol": "KRTAP5-8",
  "term_id": "UNKNOWN:0002",
  "gene": "UniProtKB:O75690",
  "term_label": "Unknown biological process",
  "gene_name": "Keratin-associated protein 5-8"
}